{
  "term_id": "GO:0006612",
  "gene_name": "Nascent polypeptide-associated complex subunit alpha-2",
  "gene": "UniProtKB:Q9H009",
  "gene_symbol": "NACA2",
  "term_label": "protein targeting to membrane"
}